{
  "gene_name": "Tripartite motif-containing protein 6",
  "term_label": "protein kinase binding",
  "gene": "UniProtKB:Q9C030",
  "gene_symbol": "TRIM6",
  "term_id": "GO:0019901"
}